regulation of dendritic cell dendrite assembly [GO:2000547] (biological process) Also known as: regulation of dendritic extension Definition: Any process that modulates the frequency, rate or extent of dendritic cell dendrite assembly. Sources: GOC:obol Subtypes: negative regulation of dendritic cell dendrite assembly [GO:2000548], GO:2000549 Relationships: is a type of regulation of plasma membrane bounded cell projection assembly [GO:0120032]; regulates dendritic cell dendrite assembly [GO:0097026]